tungsten incorporation into tungsten-molybdopterin complex [GO:0042042] (biological process) Sources: GOC:ai Relationships: is a type of metal incorporation into metallo-molybdopterin complex [GO:0042040] Definition: The incorporation of tungsten into a tungsten-molybdopterin complex.